{
  "gene": "UniProtKB:A0A0G2JNH3",
  "gene_name": "Olfactory receptor",
  "term_label": "Unknown biological process",
  "term_id": "UNKNOWN:0002",
  "gene_symbol": "LOC124905359"
}